{
  "gene": "UniProtKB:Q9H0K6",
  "term_id": "GO:0005634",
  "gene_name": "Pseudouridylate synthase PUS7L",
  "gene_symbol": "PUS7L",
  "term_label": "nucleus"
}